{
  "gene": "UniProtKB:P54845",
  "gene_symbol": "NRL",
  "term_id": "GO:0000978",
  "gene_name": "Neural retina-specific leucine zipper protein",
  "term_label": "RNA polymerase II cis-regulatory region sequence-specific DNA binding"
}